{
  "gene": "UniProtKB:Q5T8I9",
  "gene_symbol": "HENMT1",
  "term_id": "GO:0030422",
  "term_label": "siRNA processing",
  "gene_name": "Small RNA 2'-O-methyltransferase"
}